{
  "term_label": "cilium movement involved in cell motility",
  "gene": "UniProtKB:Q9P225",
  "term_id": "GO:0060294",
  "gene_symbol": "DNAH2",
  "gene_name": "Dynein axonemal heavy chain 2"
}